{
  "term_id": "GO:0030515",
  "gene_symbol": "RRP9",
  "gene": "UniProtKB:O43818",
  "term_label": "snoRNA binding",
  "gene_name": "U3 small nucleolar RNA-interacting protein 2"
}